{
  "gene_name": "Transmembrane and coiled-coil domain-containing protein 6",
  "gene": "UniProtKB:Q96DC7",
  "gene_symbol": "TMCO6",
  "term_id": "UNKNOWN:0002",
  "term_label": "Unknown biological process"
}